{
  "gene_name": "Glycerol-3-phosphate acyltransferase 1, mitochondrial",
  "gene_symbol": "GPAM",
  "term_id": "GO:0004366",
  "term_label": "glycerol-3-phosphate O-acyltransferase activity",
  "gene": "UniProtKB:Q9HCL2"
}